{
  "term_label": "ribonucleoside triphosphate phosphatase activity",
  "gene": "UniProtKB:P49961",
  "term_id": "GO:0017111",
  "gene_symbol": "ENTPD1",
  "gene_name": "Ectonucleoside triphosphate diphosphohydrolase 1"
}